cellular response to tetracycline [GO:0072746] (biological process) Definition: Any process that results in a change in state or activity of a cell (in terms of movement, secretion, enzyme production, gene expression, etc.) as a result of a tetracycline stimulus. Sources: GOC:mah Relationships: is a type of cellular response to alcohol [GO:0097306]; is a type of response to tetracycline [GO:1901326]; is a type of cellular response to ketone [GO:1901655]